{
  "term_id": "GO:0030199",
  "gene_symbol": "P3H4",
  "term_label": "collagen fibril organization",
  "gene_name": "Endoplasmic reticulum protein SC65",
  "gene": "UniProtKB:Q92791"
}